{
  "gene": "UniProtKB:P00740",
  "term_id": "GO:0007596",
  "gene_symbol": "F9",
  "term_label": "blood coagulation",
  "gene_name": "Coagulation factor IX"
}